{
  "gene_name": "Ubiquitin carboxyl-terminal hydrolase 17-like protein 10",
  "gene_symbol": "USP17L10",
  "term_id": "GO:0004843",
  "term_label": "cysteine-type deubiquitinase activity",
  "gene": "UniProtKB:C9JJH3"
}